{
  "gene_symbol": "SLC6A20",
  "term_id": "GO:0035725",
  "term_label": "sodium ion transmembrane transport",
  "gene": "UniProtKB:Q9NP91",
  "gene_name": "Sodium- and chloride-dependent transporter XTRP3"
}